{
  "gene": "UniProtKB:Q92935",
  "gene_symbol": "EXTL1",
  "gene_name": "Exostosin-like 1",
  "term_label": "acetylglucosaminyltransferase activity",
  "term_id": "GO:0008375"
}